{
  "gene_name": "Sodium_potassium_calcium exchanger 1",
  "term_id": "GO:0060292",
  "gene": "UniProtKB:O60721",
  "term_label": "long-term synaptic depression",
  "gene_symbol": "SLC24A1"
}